{
  "gene": "UniProtKB:Q9H0C2",
  "gene_symbol": "SLC25A31",
  "gene_name": "ADP_ATP translocase 4",
  "term_id": "GO:0005743",
  "term_label": "mitochondrial inner membrane"
}